{
  "gene_symbol": "AGTR1",
  "gene": "UniProtKB:P30556",
  "gene_name": "Type-1 angiotensin II receptor",
  "term_label": "kidney development",
  "term_id": "GO:0001822"
}